negative regulation of signal transduction by receptor internalization [GO:0038011] (biological process) Subtypes: negative regulation of insulin receptor signaling pathway by insulin receptor internalization [GO:0038014] Relationships: is a type of negative regulation of signal transduction [GO:0009968]; is a type of regulation of signal transduction by receptor internalization [GO:0038009] Also known as: negative regulation of signaling pathway by receptor endocytosis References: PMID:17908284, PMID:19696798 Sources: GOC:bf, GOC:signaling Definition: Any process in which internalization of a signaling receptor stops, prevents, or reduces the frequency, rate or extent of signal transduction. Receptor internalization can attenuate or reduce the strength of signaling by reducing the concentration of cell surface receptors available to ligands.